{
  "gene_name": "Atypical chemokine receptor 3",
  "term_label": "C-C chemokine binding",
  "term_id": "GO:0019957",
  "gene_symbol": "ACKR3",
  "gene": "UniProtKB:P25106"
}